{
  "gene_symbol": "PPP1R35",
  "term_id": "UNKNOWN:0001",
  "term_label": "Unknown molecular function",
  "gene_name": "Protein phosphatase 1 regulatory subunit 35",
  "gene": "UniProtKB:Q8TAP8"
}